type IV site-specific deoxyribonuclease activity [GO:0032067] (molecular function) Relationships: is a type of restriction endodeoxyribonuclease activity [GO:0015666] Also known as: type IV restriction enzyme activity References: PMID:12654995 Definition: Catalysis of the endonucleolytic cleavage of DNA in a site specific manner. Cleavage is dependent on the presence of a specific recognition site in the DNA which must be modified (e.g. methylated, hydroxymethylated, glucosyl-hydroxymethylated).